ascaroside biosynthetic process [GO:1904070] (biological process) Relationships: is a type of GO:0016138 References: PMID:25775534 Sources: GOC:TermGenie, GOC:kmv, GO_REF:0000068 Also known as: ascaroside anabolism, ascaroside biosynthesis, ascaroside formation, ascaroside synthesis Definition: The chemical reactions and pathways resulting in the formation of ascaroside.